T cell homeostasis [GO:0043029] (biological process) Also known as: T lymphocyte homeostasis, T-cell homeostasis, T-lymphocyte homeostasis Definition: The process of regulating the proliferation and elimination of T cells such that the total number of T cells within a whole or part of an organism is stable over time in the absence of an outside stimulus. Relationships: is a type of GO:0002260 Subtypes: GO:0160165 Sources: GOC:mgi_curators, ISBN:0781735149 Note: Note that this term represents the return of T cell levels to stable numbers following an immune response as well as the proliferation and elimination of T cells required to maintain stable numbers in the absence of an outside stimulus.